{
  "term_label": "Notch signaling pathway",
  "gene_name": "Neurogenic locus notch homolog protein 2",
  "gene_symbol": "NOTCH2",
  "gene": "UniProtKB:Q04721",
  "term_id": "GO:0007219"
}